regulation of type I interferon-mediated signaling pathway [GO:0060338] (biological process) Definition: Any process that modulates the rate, frequency or extent of a type I interferon-mediated signaling pathway. Sources: GOC:dph Also known as: regulation of type I interferon-mediated signalling pathway Relationships: is a type of regulation of cytokine-mediated signaling pathway [GO:0001959]; is a type of regulation of innate immune response [GO:0045088]; regulates type I interferon-mediated signaling pathway [GO:0060337] Subtypes: negative regulation of type I interferon-mediated signaling pathway [GO:0060339], GO:0060340